salicyl-alcohol beta-D-glucosyltransferase activity [GO:0050274] (molecular function) Definition: Catalysis of the reaction: salicyl alcohol + UDP-D-glucose = H+ + salicin + UDP. Sources: EC:2.4.1.172, RHEA:11512 Also known as: salicyl-alcohol b-D-glucosyltransferase activity, salicyl-alcohol glucosyltransferase activity, UDP-glucose:salicyl-alcohol beta-D-glucosyltransferase activity, UDPglucose:salicyl alcohol phenyl-glucosyltransferase activity, UDPglucose:salicyl-alcohol beta-D-glucosyltransferase activity, uridine diphosphoglucose-salicyl alcohol 2-glucosyltransferase activity Relationships: is a type of UDP-glucosyltransferase activity [GO:0035251]